{
  "gene_symbol": "RNF31",
  "gene_name": "E3 ubiquitin-protein ligase RNF31",
  "gene": "UniProtKB:Q96EP0",
  "term_id": "GO:0070530",
  "term_label": "K63-linked polyubiquitin modification-dependent protein binding"
}